{
  "gene": "UniProtKB:P51689",
  "gene_symbol": "ARSD",
  "term_label": "Unknown cellular component",
  "term_id": "UNKNOWN:0003",
  "gene_name": "Arylsulfatase D"
}